{
  "gene_symbol": "LINS1",
  "gene_name": "Protein Lines homolog 1",
  "term_id": "UNKNOWN:0003",
  "term_label": "Unknown cellular component",
  "gene": "UniProtKB:Q8NG48"
}